{
  "term_id": "UNKNOWN:0001",
  "gene": "UniProtKB:Q8NDC0",
  "term_label": "Unknown molecular function",
  "gene_name": "MAPK-interacting and spindle-stabilizing protein-like",
  "gene_symbol": "MAPK1IP1L"
}